{
  "gene_name": "Cyclin-T1",
  "term_id": "GO:0045944",
  "gene": "UniProtKB:O60563",
  "term_label": "positive regulation of transcription by RNA polymerase II",
  "gene_symbol": "CCNT1"
}